{
  "term_id": "GO:0007221",
  "gene_symbol": "MAML2",
  "gene": "UniProtKB:Q8IZL2",
  "term_label": "positive regulation of transcription of Notch receptor target",
  "gene_name": "Mastermind-like protein 2"
}